postsynaptic density membrane [GO:0098839] (cellular component) Sources: GOC:dos Definition: The membrane component of the postsynaptic density. This is the region of the postsynaptic membrane in which the population of neurotransmitter receptors involved in synaptic transmission are concentrated. Relationships: is a type of postsynaptic specialization membrane [GO:0099634]; is part of postsynaptic density [GO:0014069]